{
  "term_id": "GO:0005737",
  "gene_name": "E3 ubiquitin-protein ligase TRIM13",
  "gene_symbol": "TRIM13",
  "term_label": "cytoplasm",
  "gene": "UniProtKB:O60858"
}